{
  "gene": "UniProtKB:P49682",
  "gene_name": "C-X-C chemokine receptor type 3",
  "gene_symbol": "CXCR3",
  "term_id": "GO:0007204",
  "term_label": "positive regulation of cytosolic calcium ion concentration"
}